{
  "gene_symbol": "ZNF148",
  "term_label": "RNA polymerase II cis-regulatory region sequence-specific DNA binding",
  "gene_name": "Zinc finger protein 148",
  "gene": "UniProtKB:Q9UQR1",
  "term_id": "GO:0000978"
}